{
  "gene_name": "NADH dehydrogenase [ubiquinone] 1 beta subcomplex subunit 5, mitochondrial",
  "gene": "UniProtKB:O43674",
  "term_id": "UNKNOWN:0001",
  "term_label": "Unknown molecular function",
  "gene_symbol": "NDUFB5"
}